beta-6-sulfate-N-acetylglucosaminidase activity [GO:0052769] (molecular function) Also known as: beta-6-SO3-N-acetylglucosaminidase activity, exosulfoglycosidase activity, sulfoglycosidase activity, sulfomucin beta-6-sulfate-N-acetylglucosaminidase activity References: PMID:15716424 Sources: GOC:mengo_curators Definition: Catalysis of the glycosidic cleavage of the terminal 2-acetamido-2-deoxy-beta-D-glucopyranoside 6-sulfate (6-SO3-GlcNAc) residue from sulfomucin, a sulfated mucin derivative. Relationships: is a type of hydrolase activity, hydrolyzing O-glycosyl compounds [GO:0004553]